{
  "gene_name": "Semaphorin-3A",
  "gene_symbol": "SEMA3A",
  "gene": "UniProtKB:Q14563",
  "term_id": "GO:0071526",
  "term_label": "semaphorin-plexin signaling pathway"
}